{
  "term_label": "cytosol",
  "gene_name": "Aldo-keto reductase family 1 member A1",
  "term_id": "GO:0005829",
  "gene": "UniProtKB:P14550",
  "gene_symbol": "AKR1A1"
}